triterpenoid metabolic process [GO:0006722] (biological process) Relationships: is a type of terpenoid metabolic process [GO:0006721] Also known as: triterpenoid metabolism, triterpene metabolic process, triterpene metabolism Sources: ISBN:0198547684 Definition: The chemical reactions and pathways involving triterpenoid compounds, terpenoids with six isoprene units. Subtypes: triterpenoid biosynthetic process [GO:0016104], triterpenoid catabolic process [GO:0016105], GO:0019742, thalianol metabolic process [GO:0080003]